{
  "gene_name": "ATPase inhibitor, mitochondrial",
  "gene": "UniProtKB:Q9UII2",
  "term_label": "ATPase binding",
  "gene_symbol": "ATP5IF1",
  "term_id": "GO:0051117"
}